{
  "gene": "UniProtKB:Q7RTY1",
  "term_id": "GO:0008028",
  "gene_name": "Monocarboxylate transporter 9",
  "term_label": "monocarboxylic acid transmembrane transporter activity",
  "gene_symbol": "SLC16A9"
}